{
  "term_id": "UNKNOWN:0003",
  "gene": "UniProtKB:Q6NXP6",
  "term_label": "Unknown cellular component",
  "gene_symbol": "NOXRED1",
  "gene_name": "NADP-dependent oxidoreductase domain-containing protein 1"
}